{
  "gene_symbol": "SLITRK3",
  "term_id": "UNKNOWN:0001",
  "term_label": "Unknown molecular function",
  "gene_name": "SLIT and NTRK-like protein 3",
  "gene": "UniProtKB:O94933"
}